{
  "gene_symbol": "STRIT1",
  "gene_name": "Sarcoplasmic_endoplasmic reticulum calcium ATPase regulator DWORF",
  "term_id": "UNKNOWN:0002",
  "gene": "UniProtKB:P0DN84",
  "term_label": "Unknown biological process"
}